{
  "gene": "UniProtKB:Q13491",
  "term_label": "plasma membrane",
  "gene_name": "Neuronal membrane glycoprotein M6-b",
  "gene_symbol": "GPM6B",
  "term_id": "GO:0005886"
}